15-hydroxyprostaglandin dehydrogenase (NADP+) activity [GO:0047021] (molecular function) Relationships: is_a GO:0016616 Sources: EC:1.1.1.197, RHEA:11636 Also known as: NADP-dependent 15-hydroxyprostaglandin dehydrogenase, NADP-linked 15-hydroxyprostaglandin dehydrogenase, NADP-specific 15-hydroxyprostaglandin dehydrogenase, (13E)-(15S)-11alpha,15-dihydroxy-9-oxoprost-13-enoate:NADP+ 15-oxidoreductase activity, type II 15-hydroxyprostaglandin dehydrogenase activity Definition: Catalysis of the reaction: NADP+ + prostaglandin E(1) = 15-dehydro-prostaglandin E1 + H+ + NADPH.